symbiont-mediated suppression of host JAK-STAT cascade [GO:0039514] (biological process) References: PMID:20624917, PMID:22919663, PMID:27437422, PMID:29924996, PMID:31413201 Sources: GOC:bf, GOC:sp Relationships: is_a symbiont-mediated suppression of host signal transduction pathway [GO:0052029] Also known as: disruption by virus of host JAK-STAT cascade, down-regulation by virus of host JAK-STAT cascade, downregulation by virus of host JAK-STAT cascade, inhibition by virus of host JAK-STAT cascade, negative regulation by virus of host JAK-STAT cascade, suppression by virus of host JAK-STAT cascade Definition: A process in which a symbiont interferes with, inhibits or disrupt a JAK-STAT signal cascade in the host organism. The host is defined as the larger of the organisms involved in a symbiotic interaction. Subtypes: symbiont-mediated suppression of host JAK-STAT cascade via inhibition of host IRF9 activity [GO:0039560], symbiont-mediated suppression of host JAK-STAT cascade via inhibition of STAT activity [GO:0039562], symbiont-mediated suppression of host JAK-STAT cascade via inhibition of host TYK2 activity [GO:0039574], GO:0039576